sorocarp sorus development [GO:0048837] (biological process) Definition: The process whose specific outcome is the progression of the sorocarp sorus over time, from its formation to the mature structure. A sorocarp sorus is the spore containing structure of a sorocarp. References: PMID:4332228 Sources: GOC:devbiol, GOC:mtg_sensu Relationships: is a type of GO:0099120; is part of GO:0031154 Also known as: sorocarp sorus formation, sorocarp spore head formation, sorocarp spore head morphogenesis